mannosyl diphosphorylinositol ceramide metabolic process [GO:0006676] (biological process) Definition: The chemical reactions and pathways involving mannosyl diphosphorylinositol ceramide, any lipid with a phosphodiester bridge between an inositol residue and the ceramide group which contains two phosphoryl (-P(O)=) groups and a mannose derivative. Sources: GOC:ai Also known as: M(IP)2C metabolic process, M(IP)2C metabolism, mannosyl diphosphorylinositol ceramide metabolism Relationships: is a type of GPI anchor metabolic process [GO:0006505]; is_a inositol phosphoceramide metabolic process [GO:0006673]